{
  "term_label": "late endosome",
  "gene_name": "RING finger protein 148",
  "term_id": "GO:0005770",
  "gene": "UniProtKB:Q8N7C7",
  "gene_symbol": "RNF148"
}